{
  "term_id": "UNKNOWN:0003",
  "gene_name": "Coiled-coil domain-containing protein 200",
  "gene": "UniProtKB:A0A1B0GVQ3",
  "term_label": "Unknown cellular component",
  "gene_symbol": "CCDC200"
}